{
  "gene_symbol": "CFAP161",
  "gene": "UniProtKB:Q6P656",
  "term_id": "GO:0031514",
  "gene_name": "Cilia- and flagella-associated protein 161",
  "term_label": "motile cilium"
}